{
  "term_id": "UNKNOWN:0002",
  "term_label": "Unknown biological process",
  "gene_name": "Probable non-functional T cell receptor gamma variable 11",
  "gene_symbol": "TRGV11",
  "gene": "UniProtKB:A0A075B6L2"
}